{
  "gene_name": "Afadin",
  "gene_symbol": "AFDN",
  "term_label": "cell adhesion molecule binding",
  "gene": "UniProtKB:P55196",
  "term_id": "GO:0050839"
}